{
  "gene_symbol": "TBC1D13",
  "term_label": "intracellular protein transport",
  "term_id": "GO:0006886",
  "gene": "UniProtKB:Q9NVG8",
  "gene_name": "TBC1 domain family member 13"
}